sperm storage [GO:0046693] (biological process) Relationships: is a type of sperm competition [GO:0046692] Definition: The retention of sperm by a female following mating. Also known as: retention of sperm, sequestering of sperm, sequestration of sperm, sperm retention, sperm sequestering, sperm sequestration, storage of sperm References: PMID:10885514